{
  "gene_symbol": "ITGA4",
  "term_id": "GO:0098609",
  "term_label": "cell-cell adhesion",
  "gene_name": "Integrin alpha-4",
  "gene": "UniProtKB:P13612"
}